{
  "gene_symbol": "PTRHD1",
  "term_id": "UNKNOWN:0002",
  "term_label": "Unknown biological process",
  "gene": "UniProtKB:Q6GMV3",
  "gene_name": "Putative peptidyl-tRNA hydrolase PTRHD1"
}